{
  "gene": "UniProtKB:Q9H6Z4",
  "term_id": "GO:0006611",
  "gene_name": "Ran-binding protein 3",
  "term_label": "protein export from nucleus",
  "gene_symbol": "RANBP3"
}